symbiont-mediated perturbation of host defense response [GO:0052031] (biological process) Definition: A process in which a symbiont interferes with the ability of the host to mount a defense in response to its presence. The host is defined as the larger of the organisms involved in a symbiotic interaction. Subtypes: symbiont-mediated-mediated suppression of host tetherin activity [GO:0039587], GO:0052084, GO:0052160, symbiont-mediated perturbation of host immune response [GO:0052553], symbiont-mediated suppression of host CRISPR-cas system [GO:0098672], GO:0140415, symbiont-mediated perturbation of host opsonization [GO:0141073], symbiont-mediated suppression of host reactive oxygen species generation [GO:0141083], symbiont-mediated suppression of host neutrophil extracellular trap formation [GO:0141145], symbiont-mediated suppression of host phagosome acidification [GO:0141159] Relationships: is a type of symbiont-mediated perturbation of host process [GO:0044003] Sources: GOC:mtg_pamgo_17jul06 Also known as: modulation by organism of defense response of other organism involved in symbiotic interaction, mitigation by symbiont of host defense response, modulation by symbiont of host defense response, perturbation by symbiont of host defense response, pathogenesis